{
  "gene_symbol": "NLN",
  "term_label": "mitochondrial intermembrane space",
  "gene_name": "Neurolysin, mitochondrial",
  "term_id": "GO:0005758",
  "gene": "UniProtKB:Q9BYT8"
}